{
  "term_label": "Unknown cellular component",
  "gene_symbol": "RAB3IL1",
  "term_id": "UNKNOWN:0003",
  "gene": "UniProtKB:Q8TBN0",
  "gene_name": "Guanine nucleotide exchange factor for Rab-3A"
}